intracellularly ligand-gated monoatomic ion channel activity [GO:0005217] (molecular function) Relationships: is a type of ligand-gated monoatomic ion channel activity [GO:0015276] Sources: GOC:mtg_transport, ISBN:0815340729 Subtypes: GO:0005221, intracellularly gated calcium channel activity [GO:0015278], intracellularly phosphatidylinositol-3,5-bisphosphate-gated monatomic cation channel activity [GO:0097682], GO:0099142 Also known as: intracellular ligand-gated ion channel activity, intracellular ligand-gated monoatomic ion channel activity Definition: Enables the transmembrane transfer of an ion by a channel that opens when a specific intracellular ligand has been bound by the channel complex or one of its constituent parts.